negative regulation of retinal cone cell fate specification [GO:0009998] (biological process) Sources: GOC:go_curators Definition: Any process that restricts, stops or prevents a cell from specifying into a retinal cone cell. Also known as: down regulation of retinal cone cell fate specification, down-regulation of retinal cone cell fate specification, downregulation of retinal cone cell fate specification, negative regulation of retina cone cell fate specification, suppression of retina cone cell fate, suppression of retinal cone cell fate, inhibition of retinal cone cell fate specification Relationships: is_a negative regulation of cell fate specification [GO:0009996]; is a type of regulation of retinal cone cell fate specification [GO:0042673]; is_a negative regulation of retinal cone cell fate commitment [GO:0060226]; negatively regulates retinal cone cell fate specification [GO:0042672]